NAD transport [GO:0043132] (biological process) Sources: GOC:jl Also known as: NAD (oxidized) transport, NAD (reduced) transport, NADH transport, nicotinamide adenine dinucleotide transport, oxidized NAD transport, oxidized nicotinamide adenine dinucleotide transport, reduced NAD transport, reduced nicotinamide adenine dinucleotide transport Subtypes: NAD transmembrane transport [GO:0035352] Relationships: is a type of adenine nucleotide transport [GO:0051503] Definition: The directed movement of nicotinamide adenine dinucleotide into, out of or within a cell, or between cells, by means of some agent such as a transporter or pore; transport may be of either the oxidized form, NAD, or the reduced form, NADH.